{
  "gene": "UniProtKB:P49767",
  "term_id": "GO:0048010",
  "term_label": "vascular endothelial growth factor receptor signaling pathway",
  "gene_symbol": "VEGFC",
  "gene_name": "Vascular endothelial growth factor C"
}